negative regulation of cargo loading into COPII-coated vesicle [GO:1901303] (biological process) Definition: Any process that stops, prevents or reduces the frequency, rate or extent of cargo loading into a COPII-coated vesicle. Relationships: is_a GO:0032387; is a type of regulation of cargo loading into COPII-coated vesicle [GO:1901301]; negatively regulates GO:0090110 Also known as: down regulation of cargo loading into COPII vesicle, down regulation of cargo loading into COPII-coated vesicle, down regulation of cargo selection into COPII-coated vesicle, down-regulation of cargo loading into COPII vesicle, down-regulation of cargo loading into COPII-coated vesicle, down-regulation of cargo selection into COPII-coated vesicle, downregulation of cargo loading into COPII vesicle, downregulation of cargo loading into COPII-coated vesicle, downregulation of cargo selection into COPII-coated vesicle, inhibition of cargo loading into COPII vesicle, inhibition of cargo selection into COPII-coated vesicle, inhibition of protein sorting into COPII-coated vesicles, negative regulation of cargo loading into COPII vesicle, negative regulation of cargo selection into COPII-coated vesicle, inhibition of COPII vesicle protein binding, inhibition of cargo loading into COPII-coated vesicle, down regulation of COPII coat-cargo complex assembly, down-regulation of COPII coat-cargo complex assembly, downregulation of COPII coat-cargo complex assembly, inhibition of COPII coat-cargo complex assembly, negative regulation of COPII coat-cargo complex assembly References: PMID:15899885 Sources: GOC:TermGenie, GOC:lb